{
  "gene_name": "Cytochrome b5 domain-containing protein 1",
  "gene": "UniProtKB:Q6P9G0",
  "gene_symbol": "CYB5D1",
  "term_label": "Unknown molecular function",
  "term_id": "UNKNOWN:0001"
}